{
  "gene_symbol": "KLF18",
  "term_id": "GO:0005634",
  "gene": "UniProtKB:A0A0U1RQI7",
  "term_label": "nucleus",
  "gene_name": "Kruppel-like factor 18"
}